{
  "term_label": "positive regulation of transcription by RNA polymerase III",
  "term_id": "GO:0045945",
  "gene_symbol": "ICE2",
  "gene": "UniProtKB:Q659A1",
  "gene_name": "Little elongation complex subunit 2"
}